cellular response to actinomycin D [GO:0072717] (biological process) Definition: Any process that results in a change in state or activity of a cell (in terms of movement, secretion, enzyme production, gene expression, etc.) as a result of an actinomycin D stimulus. Relationships: is_a cellular response to antibiotic [GO:0071236]; is a type of GO:0072716; is a type of GO:1901699; is a type of cellular response to oxygen-containing compound [GO:1901701] Sources: GOC:mah